{
  "term_label": "Unknown biological process",
  "gene_name": "Centromere protein V-like protein 3",
  "term_id": "UNKNOWN:0002",
  "gene": "UniProtKB:A0A0U1RRI6",
  "gene_symbol": "CENPVL3"
}